{
  "term_id": "GO:0034475",
  "gene": "UniProtKB:Q9NPD3",
  "term_label": "U4 snRNA 3'-end processing",
  "gene_symbol": "EXOSC4",
  "gene_name": "Exosome complex component RRP41"
}